{
  "gene_symbol": "SLC28A3",
  "term_id": "GO:0015864",
  "term_label": "pyrimidine nucleoside transport",
  "gene": "UniProtKB:Q9HAS3",
  "gene_name": "Solute carrier family 28 member 3"
}